{
  "term_label": "peptidase activator activity",
  "gene": "UniProtKB:Q9UKZ9",
  "gene_symbol": "PCOLCE2",
  "term_id": "GO:0016504",
  "gene_name": "Procollagen C-endopeptidase enhancer 2"
}